thiaminase activity [GO:0050334] (molecular function) Sources: EC:3.5.99.2, RHEA:17509 Definition: Catalysis of the reaction: H2O + thiamine = 4-amino-5-hydroxymethyl-2-methylpyrimidine + 5-(2-hydroxyethyl)-4-methylthiazole + H+. Relationships: is a type of hydrolase activity, acting on carbon-nitrogen (but not peptide) bonds [GO:0016810] Also known as: thiaminase II activity